{
  "gene": "UniProtKB:P01135",
  "term_id": "GO:0008284",
  "term_label": "positive regulation of cell population proliferation",
  "gene_name": "Protransforming growth factor alpha",
  "gene_symbol": "TGFA"
}